{
  "term_label": "RNA polymerase II cis-regulatory region sequence-specific DNA binding",
  "term_id": "GO:0000978",
  "gene": "UniProtKB:P10243",
  "gene_symbol": "MYBL1",
  "gene_name": "Myb-related protein A"
}